{
  "gene_symbol": "UTP6",
  "gene": "UniProtKB:Q9NYH9",
  "term_label": "small-subunit processome",
  "term_id": "GO:0032040",
  "gene_name": "U3 small nucleolar RNA-associated protein 6 homolog"
}